Ala-tRNA(Thr) deacylase activity [GO:0106105] (molecular function) Definition: Catalysis of the reaction: L-alanyl-tRNA(Thr) + H2O = tRNA(Thr) + L-alanine + H+. Also known as: L-alanyl-tRNA(Thr) deacylase Relationships: is a type of GO:0002161 References: PMID:29410408 Sources: RHEA:17793